{
  "gene_name": "Kelch-like protein 10",
  "gene_symbol": "KLHL10",
  "term_id": "GO:0005737",
  "gene": "UniProtKB:Q6JEL2",
  "term_label": "cytoplasm"
}